{
  "gene_name": "Palmitoyltransferase ZDHHC6",
  "term_id": "GO:0019706",
  "gene_symbol": "ZDHHC6",
  "gene": "UniProtKB:Q9H6R6",
  "term_label": "protein-cysteine S-palmitoyltransferase activity"
}